{
  "gene": "UniProtKB:Q9BZE1",
  "gene_name": "Large ribosomal subunit protein mL37",
  "gene_symbol": "MRPL37",
  "term_id": "UNKNOWN:0001",
  "term_label": "Unknown molecular function"
}